growing cell tip [GO:0035838] (cellular component) Sources: GOC:mah Definition: The region at either end of the longest axis of a cylindrical or elongated cell, where polarized growth occurs. Also known as: growing cell end Subtypes: old growing cell tip [GO:0035840], new growing cell tip [GO:0035841], pollen tube tip [GO:0090404] Relationships: is_a GO:0030427; is a type of cell tip [GO:0051286]